{
  "gene_name": "Rhophilin-1",
  "term_id": "GO:0051497",
  "term_label": "negative regulation of stress fiber assembly",
  "gene_symbol": "RHPN1",
  "gene": "UniProtKB:Q8TCX5"
}